{
  "gene": "UniProtKB:Q96N95",
  "term_id": "GO:0000978",
  "term_label": "RNA polymerase II cis-regulatory region sequence-specific DNA binding",
  "gene_symbol": "ZNF396",
  "gene_name": "Zinc finger protein 396"
}